{
  "gene_name": "Fibroblast growth factor-binding protein 2",
  "term_id": "UNKNOWN:0003",
  "gene_symbol": "FGFBP2",
  "gene": "UniProtKB:Q9BYJ0",
  "term_label": "Unknown cellular component"
}